{
  "term_label": "cysteine-type endopeptidase inhibitor activity",
  "gene_symbol": "PTTG1",
  "gene": "UniProtKB:O95997",
  "gene_name": "Securin",
  "term_id": "GO:0004869"
}